{
  "gene": "UniProtKB:A0A5F9Z9Y6",
  "gene_symbol": "A0A5F9Z9Y6",
  "gene_name": "Immunoglobulin subtype domain-containing protein",
  "term_id": "GO:0005886",
  "term_label": "plasma membrane"
}